regulation of stress-activated MAPK cascade [GO:0032872] (biological process) Also known as: regulation of p38 MAPK signaling, regulation of p38 MAPK signalling, regulation of stress-activated MAPK signaling pathway, regulation of stress-activated MAPK signalling pathway, regulation of stress-activated MAPKKK cascade, regulation of stress-activated MAPKKK signaling pathway, regulation of stress-activated MAPKKK signalling pathway Sources: GOC:mah Relationships: is a type of regulation of MAPK cascade [GO:0043408]; is a type of GO:0070302; regulates stress-activated MAPK cascade [GO:0051403] Subtypes: GO:0032873, positive regulation of stress-activated MAPK cascade [GO:0032874], regulation of cell integrity MAPK cascade [GO:1903137] Definition: Any process that modulates the frequency, rate or extent of signal transduction mediated by the stress-activated MAPK cascade.